{
  "term_label": "adherens junction",
  "gene": "UniProtKB:Q96AP7",
  "term_id": "GO:0005912",
  "gene_symbol": "ESAM",
  "gene_name": "Endothelial cell-selective adhesion molecule"
}